{
  "term_label": "tRNA wobble position uridine thiolation",
  "gene_name": "Cytoplasmic tRNA 2-thiolation protein 2",
  "term_id": "GO:0002143",
  "gene": "UniProtKB:Q2VPK5",
  "gene_symbol": "CTU2"
}